{
  "gene_name": "Matrix metalloproteinase-16",
  "gene": "UniProtKB:P51512",
  "gene_symbol": "MMP16",
  "term_id": "GO:0001501",
  "term_label": "skeletal system development"
}